{
  "term_id": "GO:0006606",
  "gene": "UniProtKB:Q8TEX9",
  "gene_symbol": "IPO4",
  "term_label": "protein import into nucleus",
  "gene_name": "Importin-4"
}